response to oxygen-glucose deprivation [GO:0090649] (biological process) References: PMID:21525936 Sources: GOC:sl Also known as: response to OGD Definition: Any process that results in a change in state or activity of a cell or an organism (in terms of movement, secretion, enzyme production, gene expression, etc.) as a result of the deprivation of oxygen and glucose. Relationships: is a type of response to nutrient levels [GO:0031667]; is a type of response to decreased oxygen levels [GO:0036293] Subtypes: cellular response to oxygen-glucose deprivation [GO:0090650]